{
  "term_id": "GO:0043495",
  "term_label": "protein-membrane adaptor activity",
  "gene_name": "Guided entry of tail-anchored proteins factor 1",
  "gene": "UniProtKB:O00258",
  "gene_symbol": "GET1"
}